{
  "gene_symbol": "CATSPER2",
  "term_label": "Unknown molecular function",
  "gene": "UniProtKB:Q96P56",
  "term_id": "UNKNOWN:0001",
  "gene_name": "Cation channel sperm-associated protein 2"
}